olfactory placode development [GO:0071698] (biological process) Sources: GOC:mah Relationships: is a type of GO:0071696 Definition: The progression of the olfactory placode over time from its initial formation until its mature state. The olfactory placode is a thickening of the neural ectoderm in the head region of the vertebrate embryo which develops into the olfactory region of the nasal cavity.